{
  "gene_name": "U2 small nuclear ribonucleoprotein B''",
  "term_label": "U1 snRNA binding",
  "gene_symbol": "SNRPB2",
  "gene": "UniProtKB:P08579",
  "term_id": "GO:0030619"
}